{
  "gene_symbol": "NRG1",
  "term_id": "GO:0038130",
  "gene_name": "Pro-neuregulin-1, membrane-bound isoform",
  "term_label": "ERBB4 signaling pathway",
  "gene": "UniProtKB:Q02297"
}